{
  "gene_name": "Protein crumbs homolog 1",
  "gene_symbol": "CRB1",
  "term_id": "GO:0032991",
  "gene": "UniProtKB:P82279",
  "term_label": "protein-containing complex"
}